{
  "gene_name": "Integrator complex subunit 3",
  "term_id": "UNKNOWN:0002",
  "term_label": "Unknown biological process",
  "gene": "UniProtKB:Q68E01",
  "gene_symbol": "INTS3"
}